{
  "gene": "UniProtKB:O75152",
  "term_id": "GO:0003729",
  "term_label": "mRNA binding",
  "gene_name": "Zinc finger CCCH domain-containing protein 11A",
  "gene_symbol": "ZC3H11A"
}